{
  "term_label": "cell adhesion",
  "gene": "UniProtKB:Q9HCL0",
  "gene_name": "Protocadherin-18",
  "gene_symbol": "PCDH18",
  "term_id": "GO:0007155"
}